{
  "term_label": "SUMO ligase activity",
  "gene_symbol": "KIAA1586",
  "term_id": "GO:0061665",
  "gene_name": "E3 SUMO-protein ligase KIAA1586",
  "gene": "UniProtKB:Q9HCI6"
}